benzylpenicillin catabolic process [GO:1901087] (biological process) Also known as: benzylpenicillin breakdown, benzylpenicillin catabolism, benzylpenicillin degradation, penicillin G breakdown, penicillin G catabolic process, penicillin G catabolism, penicillin G degradation Definition: The chemical reactions and pathways resulting in the breakdown of benzylpenicillin. Relationships: is a type of penicillin catabolic process [GO:0042317]; is a type of benzylpenicillin metabolic process [GO:1901086] Sources: GOC:TermGenie, GOC:yaf, UniPathway:UPA00149